spinal cord development [GO:0021510] (biological process) Definition: The process whose specific outcome is the progression of the spinal cord over time, from its formation to the mature structure. The spinal cord primarily conducts sensory and motor nerve impulses between the brain and the peripheral nervous tissues. Sources: GOC:cls, GOC:dgh, GOC:dph, GOC:jid, GO_REF:0000021 Relationships: is a type of GO:0048856; is part of central nervous system development [GO:0007417]